{
  "term_id": "UNKNOWN:0003",
  "gene": "UniProtKB:O15034",
  "gene_symbol": "RIMBP2",
  "gene_name": "RIMS-binding protein 2",
  "term_label": "Unknown cellular component"
}